{
  "term_label": "plasma membrane",
  "gene_symbol": "ADCY1",
  "term_id": "GO:0005886",
  "gene_name": "Adenylate cyclase type 1",
  "gene": "UniProtKB:Q08828"
}